{
  "gene_name": "T-complex protein 1 subunit eta",
  "gene_symbol": "CCT7",
  "gene": "UniProtKB:Q99832",
  "term_label": "protein folding",
  "term_id": "GO:0006457"
}